{
  "term_label": "Unknown cellular component",
  "gene_symbol": "CEMIP2",
  "gene": "UniProtKB:Q9UHN6",
  "term_id": "UNKNOWN:0003",
  "gene_name": "Cell surface hyaluronidase"
}